{
  "gene_symbol": "TXNIP",
  "gene": "UniProtKB:Q9H3M7",
  "term_label": "cytoplasm",
  "term_id": "GO:0005737",
  "gene_name": "Thioredoxin-interacting protein"
}